{
  "gene_name": "Pericentriolar material 1 protein",
  "gene": "UniProtKB:Q15154",
  "term_label": "protein localization to centrosome",
  "gene_symbol": "PCM1",
  "term_id": "GO:0071539"
}